ganglion maturation [GO:0061553] (biological process) Relationships: is a type of anatomical structure maturation [GO:0071695]; is part of ganglion development [GO:0061548] Definition: A developmental process, independent of morphogenetic (shape) change, that is required for ganglion to attain its fully functional state. Sources: GOC:dph Subtypes: cranial ganglion maturation [GO:0061558] Also known as: ganglia maturation